{
  "gene": "UniProtKB:Q9P2F8",
  "gene_name": "Signal-induced proliferation-associated 1-like protein 2",
  "term_id": "GO:0098978",
  "gene_symbol": "SIPA1L2",
  "term_label": "glutamatergic synapse"
}